{
  "gene": "UniProtKB:O15020",
  "gene_name": "Spectrin beta chain, non-erythrocytic 2",
  "gene_symbol": "SPTBN2",
  "term_label": "plasma membrane",
  "term_id": "GO:0005886"
}